{
  "term_label": "receptor complex",
  "term_id": "GO:0043235",
  "gene_symbol": "RAMP2",
  "gene_name": "Receptor activity-modifying protein 2",
  "gene": "UniProtKB:O60895"
}